regulation of intrinsic apoptotic signaling pathway in response to DNA damage by p53 class mediator [GO:1902165] (biological process) Also known as: regulation of DNA damage response, signal transduction by p53 class mediator resulting in induction of apoptosis References: PMID:17719541 Sources: GOC:TermGenie Subtypes: negative regulation of intrinsic apoptotic signaling pathway in response to DNA damage by p53 class mediator [GO:1902166], positive regulation of intrinsic apoptotic signaling pathway in response to DNA damage by p53 class mediator [GO:1902167] Definition: Any process that modulates the frequency, rate or extent of intrinsic apoptotic signaling pathway in response to DNA damage by p53 class mediator. Relationships: is a type of regulation of intrinsic apoptotic signaling pathway in response to DNA damage [GO:1902229]; is a type of GO:1902253; regulates intrinsic apoptotic signaling pathway in response to DNA damage by p53 class mediator [GO:0042771]